cell differentiation involved in metanephros development [GO:0072202] (biological process) Subtypes: GO:0003337, metanephric mesenchymal cell differentiation [GO:0072162], GO:0072209, metanephric DCT cell differentiation [GO:0072240], metanephric juxtaglomerulus cell differentiation [GO:0072251], GO:0072257, metanephric interstitial fibroblast differentiation [GO:0072258], mesenchymal stem cell differentiation involved in metanephric nephron morphogenesis [GO:0072281], GO:0072312 Definition: The process in which relatively unspecialized cells acquire specialized structural and/or functional features that characterize the cells of the metanephros as it progresses from its formation to the mature state. Sources: GOC:mah, GOC:mtg_kidney_jan10 Relationships: is a type of cell differentiation involved in kidney development [GO:0061005]; is part of metanephros development [GO:0001656]